X chromosome [GO:0000805] (cellular component) Relationships: is a type of sex chromosome [GO:0000803] References: PMID:20622855 Sources: GOC:mah, GOC:mr, ISBN:0582227089, Wikipedia:XY_sex-determination_system Definition: The sex chromosome present in both sexes of species in which the male is the heterogametic sex. Two copies of the X chromosome are present in each somatic cell of females and one copy is present in males. Subtypes: Barr body [GO:0001740]